epithelial cell proliferation involved in mammary gland duct elongation [GO:0060750] (biological process) Sources: GOC:dph Relationships: is a type of mammary gland epithelial cell proliferation [GO:0033598]; is part of branch elongation involved in mammary gland duct branching [GO:0060751] Definition: The multiplication or reproduction of mammary gland branch epithelial cells, resulting in the elongation of the branch. The mammary gland branch differs from the bud in that it is not the initial curved portion of the outgrowth.